{
  "gene_symbol": "DKC1",
  "gene": "UniProtKB:O60832",
  "term_label": "box H/ACA sno(s)RNA 3'-end processing",
  "term_id": "GO:0000495",
  "gene_name": "H_ACA ribonucleoprotein complex subunit DKC1"
}